{
  "gene_symbol": "RNF128",
  "gene": "UniProtKB:Q8TEB7",
  "term_label": "endoplasmic reticulum",
  "term_id": "GO:0005783",
  "gene_name": "E3 ubiquitin-protein ligase RNF128"
}